{
  "gene": "UniProtKB:O60939",
  "term_id": "GO:0017080",
  "term_label": "sodium channel regulator activity",
  "gene_name": "Sodium channel subunit beta-2",
  "gene_symbol": "SCN2B"
}